{
  "gene_name": "DDB1- and CUL4-associated factor 4-like protein 2",
  "term_id": "GO:0080008",
  "gene": "UniProtKB:Q8NA75",
  "term_label": "Cul4-RING E3 ubiquitin ligase complex",
  "gene_symbol": "DCAF4L2"
}